TRAIL receptor activity [GO:0036463] (molecular function) Relationships: is a type of death receptor activity [GO:0005035]; is part of TRAIL-activated apoptotic signaling pathway [GO:0036462]; has part TRAIL binding [GO:0045569] Definition: Combining with the ligand TRAIL (tumor necrosis factor-related apoptosis-inducing ligand) and transmitting the signal from one side of the plasma membrane to the other to initiate apoptotic cell death. Also known as: tumor necrosis factor-related apoptosis-inducing ligand receptor Sources: GOC:PARL, GOC:bf